betaine reductase activity [GO:0033795] (molecular function) Relationships: is a type of oxidoreductase activity, acting on X-H and Y-H to form an X-Y bond, with a disulfide as acceptor [GO:0050485] Also known as: acetyl-phosphate trimethylamine:thioredoxin disulfide oxidoreductase (N,N,N-trimethylglycine-forming) activity Definition: Catalysis of the reaction: [thioredoxin]-disulfide + acetyl phosphate + H2O + trimethylamine = [thioredoxin]-dithiol + glycine betaine + H+ + phosphate. Sources: RHEA:11848